{
  "gene": "UniProtKB:Q9NTZ6",
  "gene_name": "RNA-binding protein 12",
  "term_label": "regulation of RNA splicing",
  "term_id": "GO:0043484",
  "gene_symbol": "RBM12"
}